phosphatidylglycerol binding [GO:1901611] (molecular function) Relationships: is a type of phospholipid binding [GO:0005543]; is a type of anion binding [GO:0043168] Sources: GOC:TermGenie, GOC:kmv Subtypes: cardiolipin binding [GO:1901612] Definition: Binding to phosphatidylglycerol.